succinyl-diaminopimelate desuccinylase activity [GO:0009014] (molecular function) Relationships: is a type of hydrolase activity, acting on carbon-nitrogen (but not peptide) bonds, in linear amides [GO:0016811] Sources: EC:3.5.1.18, RHEA:22608 Also known as: N-succinyl-L-alpha,epsilon-diaminopimelic acid deacylase activity, N-succinyl-LL-2,6-diaminoheptanedioate amidohydrolase activity Definition: Catalysis of the reaction: N-succinyl-LL-2,6-diaminopimelate + H2O = LL-2,6-diaminopimelate + succinate.